{
  "term_label": "Unknown biological process",
  "gene_symbol": "DCBLD1",
  "gene_name": "Discoidin, CUB and LCCL domain-containing protein 1",
  "gene": "UniProtKB:Q8N8Z6",
  "term_id": "UNKNOWN:0002"
}